{
  "gene_name": "Olfactory receptor 8B3",
  "gene_symbol": "OR8B3",
  "term_label": "G protein-coupled receptor signaling pathway",
  "term_id": "GO:0007186",
  "gene": "UniProtKB:Q8NGG8"
}